alkenylglycerophosphocholine hydrolase activity [GO:0047408] (molecular function) Sources: EC:3.3.2.2, MetaCyc:3.3.2.2-RXN Definition: Catalysis of the reaction: H2O + 1-(1-alkenyl)-sn-glycero-3-phosphocholine = L-1-glycero-3-phosphocholine + an aldehyde. Also known as: 1-(1-alkenyl)-sn-glycero-3-phosphocholine aldehydohydrolase activity, lysoplasmalogenase activity Relationships: is a type of GO:0016803